glutamate decarboxylase activity [GO:0004351] (molecular function) Definition: Catalysis of the reaction: L-glutamate = 4-aminobutanoate + CO2. Also known as: aspartic alpha-decarboxylase, L-aspartate-alpha-decarboxylase activity, L-glutamate 1-carboxy-lyase (4-aminobutanoate-forming), L-glutamate 1-carboxy-lyase activity, L-glutamate alpha-decarboxylase activity, L-glutamic acid decarboxylase activity, L-glutamic decarboxylase activity, cysteic acid decarboxylase activity, gamma-glutamate decarboxylase activity Sources: EC:4.1.1.15 Relationships: is a type of carboxy-lyase activity [GO:0016831]